{
  "gene_symbol": "DGUOK",
  "gene_name": "Deoxyguanosine kinase, mitochondrial",
  "gene": "UniProtKB:Q16854",
  "term_label": "mitochondrion",
  "term_id": "GO:0005739"
}